negative regulation of gibberellic acid mediated signaling pathway [GO:0009938] (biological process) Relationships: is a type of GO:0009937; is a type of negative regulation of signal transduction [GO:0009968]; negatively regulates gibberellic acid mediated signaling pathway [GO:0009740] Definition: Any process that stops, prevents, or reduces the frequency, rate or extent of gibberellic acid mediated signaling activity. Sources: GOC:sm Also known as: down regulation of gibberellic acid mediated signaling, down-regulation of gibberellic acid mediated signaling, downregulation of gibberellic acid mediated signaling, negative regulation of gibberellic acid mediated signalling, inhibition of gibberellic acid mediated signaling